activation of monopolar cell growth [GO:0051522] (biological process) Sources: GOC:ai Relationships: is a type of GO:0051515 Definition: Any process that initiates the inactive process of monopolar cell growth, polarized growth from one end of a cell.